microtubule anchoring [GO:0034453] (biological process) Relationships: is a type of microtubule cytoskeleton organization [GO:0000226] Definition: Any process in which a microtubule is maintained in a specific location in a cell. Sources: GOC:mah Subtypes: GO:0072393, microtubule anchoring at cell cortex of cell tip [GO:0106007]